{
  "gene_name": "Disco-interacting protein 2 homolog C",
  "gene_symbol": "DIP2C",
  "term_id": "UNKNOWN:0003",
  "term_label": "Unknown cellular component",
  "gene": "UniProtKB:Q9Y2E4"
}